{
  "term_id": "GO:0030866",
  "gene_name": "Formin-like protein 3",
  "gene_symbol": "FMNL3",
  "term_label": "cortical actin cytoskeleton organization",
  "gene": "UniProtKB:Q8IVF7"
}